lysophosphatidic acid phosphatase activity [GO:0052642] (molecular function) Definition: Catalysis of the reaction: lysophosphatidic acid + H2O = phosphate + monoacylglycerol. Also known as: 1-acyl-sn-glycerol 3-phosphatase activity, 2-lysophosphatidate phosphatase activity, LPA phosphatase activity, lysophosphatidate phosphatase activity References: PMID:20045079, PMID:7966317 Relationships: is_a phosphatase activity [GO:0016791]